{
  "gene_name": "Nuclear receptor coactivator 2",
  "term_id": "GO:0016922",
  "term_label": "nuclear receptor binding",
  "gene_symbol": "NCOA2",
  "gene": "UniProtKB:Q15596"
}